positive regulation of vitellogenesis [GO:1903188] (biological process) Definition: Any process that activates or increases the frequency, rate or extent of vitellogenesis. Relationships: is a type of GO:0051130; is a type of positive regulation of multicellular organismal process [GO:0051240]; is a type of regulation of vitellogenesis [GO:1903186]; RO_0002213 vitellogenesis [GO:0007296] References: PMID:19467235 Sources: GOC:TermGenie, GOC:mr, GO_REF:0000058 Also known as: positive regulation of yolk production, up regulation of vitellogenesis, up regulation of yolk production, up-regulation of vitellogenesis, up-regulation of yolk production, upregulation of vitellogenesis, upregulation of yolk production, activation of vitellogenesis, activation of yolk production